{
  "term_id": "UNKNOWN:0002",
  "gene_symbol": "GARIN5B",
  "gene": "UniProtKB:Q8N5Q1",
  "term_label": "Unknown biological process",
  "gene_name": "Golgi-associated RAB2 interactor protein 5B"
}